{
  "gene": "UniProtKB:P41597",
  "gene_symbol": "CCR2",
  "term_id": "GO:0060326",
  "term_label": "cell chemotaxis",
  "gene_name": "C-C chemokine receptor type 2"
}